{
  "term_id": "UNKNOWN:0002",
  "gene_name": "Rho guanine nucleotide exchange factor 35",
  "gene": "UniProtKB:A5YM69",
  "gene_symbol": "ARHGEF35",
  "term_label": "Unknown biological process"
}